{
  "term_id": "GO:0005886",
  "gene": "UniProtKB:O43315",
  "gene_name": "Aquaporin-9",
  "gene_symbol": "AQP9",
  "term_label": "plasma membrane"
}